tubular endosome [GO:0097422] (cellular component) References: PMID:11896161 Sources: NIF_Subcellular:sao1570660411, NIF_Subcellular:sao694815499 Relationships: is a type of GO:0110165; is part of GO:0005768 Definition: A network of fine tubules in the vicinity of the Golgi complex and around the centriole. Also known as: coated tip